positive regulation of anther dehiscence [GO:0120195] (biological process) References: PMID:30911018 Sources: GOC:lr Relationships: is a type of regulation of anther dehiscence [GO:0120194]; is a type of positive regulation of reproductive process [GO:2000243]; positively regulates anther dehiscence [GO:0009901] Definition: Any process that activates or increases the frequency, rate or extent of anther dehiscence.